{
  "gene": "UniProtKB:P47872",
  "gene_symbol": "SCTR",
  "term_label": "secretin receptor activity",
  "gene_name": "Secretin receptor",
  "term_id": "GO:0015055"
}